{
  "gene": "UniProtKB:Q9Y546",
  "gene_name": "Leucine-rich repeat-containing protein 42",
  "gene_symbol": "LRRC42",
  "term_id": "UNKNOWN:0003",
  "term_label": "Unknown cellular component"
}